positive regulation of steroid biosynthetic process [GO:0010893] (BP) Definition: Any process that increases the frequency, rate or extent of the chemical reactions and pathways resulting in the formation of steroids, compounds with a 1,2,cyclopentanoperhydrophenanthrene nucleus. Relationships: is a type of positive regulation of steroid metabolic process [GO:0045940]; is a type of positive regulation of lipid biosynthetic process [GO:0046889]; is a type of regulation of steroid biosynthetic process [GO:0050810]; positively regulates steroid biosynthetic process [GO:0006694] Sources: GOC:tb Subtypes: GO:0060557, GO:0070859, GO:0090031, GO:0106120, positive regulation of helvolic acid biosynthetic process [GO:1900842], positive regulation of androst-4-ene-3,17-dione biosynthetic process [GO:1903456], positive regulation of estrogen biosynthetic process [GO:1904078], positive regulation of progesterone biosynthetic process [GO:2000184], GO:2000488